{
  "term_label": "Unknown cellular component",
  "gene_symbol": "ZNF280A",
  "gene_name": "Zinc finger protein 280A",
  "term_id": "UNKNOWN:0003",
  "gene": "UniProtKB:P59817"
}